G protein-coupled opioid receptor activity [GO:0004985] (molecular function) Definition: Combining with an opioid (any narcotic derived from or resembling opium), and transmitting the signal across the membrane by activating an associated G-protein. Relationships: is_a G protein-coupled receptor activity [GO:0004930]; BFO_0000050 G protein-coupled opioid receptor signaling pathway [GO:0038003] Also known as: opioid receptor activity References: PMID:20494127 Sources: GOC:ai, GOC:bf Subtypes: GO:0001626, beta-endorphin receptor activity [GO:0004979], GO:0038046, GO:0038047, GO:0038048